{
  "term_label": "RNA polymerase II cis-regulatory region sequence-specific DNA binding",
  "gene_symbol": "JUNB",
  "gene_name": "Transcription factor JunB",
  "gene": "UniProtKB:P17275",
  "term_id": "GO:0000978"
}